{
  "gene_name": "Mitochondrial assembly of ribosomal large subunit protein 1",
  "term_id": "GO:0090071",
  "term_label": "negative regulation of ribosome biogenesis",
  "gene": "UniProtKB:Q96EH3",
  "gene_symbol": "MALSU1"
}